{
  "term_label": "cytoplasm",
  "gene": "UniProtKB:P37840",
  "gene_symbol": "SNCA",
  "gene_name": "Alpha-synuclein",
  "term_id": "GO:0005737"
}